cardiac muscle cell differentiation [GO:0055007] (biological process) Sources: GOC:devbiol, GOC:mtg_heart Relationships: is a type of cardiocyte differentiation [GO:0035051]; is a type of GO:0051146; is part of GO:0048738 Regulation: regulated by regulation of cardiac muscle cell differentiation [GO:2000725]; negatively regulated by negative regulation of cardiac muscle cell differentiation [GO:2000726]; positively regulated by positive regulation of cardiac muscle cell differentiation [GO:2000727] Also known as: cardiomyocyte differentiation, heart muscle cell differentiation Subtypes: atrial cardiac muscle cell differentiation [GO:0055011], ventricular cardiac muscle cell differentiation [GO:0055012], cardiac pacemaker cell differentiation [GO:0060920], His-Purkinje system cell differentiation [GO:0060932] Definition: The process in which a cardiac muscle precursor cell acquires specialized features of a cardiac muscle cell. Cardiac muscle cells are striated muscle cells that are responsible for heart contraction.